{
  "gene_symbol": "UNC13D",
  "term_label": "secretion",
  "term_id": "GO:0046903",
  "gene_name": "Protein unc-13 homolog D",
  "gene": "UniProtKB:Q70J99"
}